{
  "term_id": "GO:0019678",
  "term_label": "propionate metabolic process, methylmalonyl pathway",
  "gene": "UniProtKB:P22033",
  "gene_name": "Methylmalonyl-CoA mutase, mitochondrial",
  "gene_symbol": "MMUT"
}